{
  "term_label": "mitochondrial outer membrane",
  "gene_symbol": "MGARP",
  "gene_name": "Protein MGARP",
  "gene": "UniProtKB:Q8TDB4",
  "term_id": "GO:0005741"
}